{
  "gene_symbol": "CATSPERE",
  "term_id": "GO:0097228",
  "gene": "UniProtKB:Q5SY80",
  "gene_name": "Cation channel sperm-associated auxiliary subunit epsilon",
  "term_label": "sperm principal piece"
}